{
  "term_id": "GO:0031490",
  "gene": "UniProtKB:Q92793",
  "gene_name": "CREB-binding protein",
  "gene_symbol": "CREBBP",
  "term_label": "chromatin DNA binding"
}